{
  "term_label": "protein serine/threonine kinase activity",
  "term_id": "GO:0004674",
  "gene_symbol": "SMG1",
  "gene_name": "Serine_threonine-protein kinase SMG1",
  "gene": "UniProtKB:Q96Q15"
}